{
  "term_id": "UNKNOWN:0003",
  "gene": "UniProtKB:Q9BQ75",
  "gene_name": "Protein CMSS1",
  "gene_symbol": "CMSS1",
  "term_label": "Unknown cellular component"
}